{
  "term_label": "cell differentiation",
  "gene_name": "Protein PRRC2A",
  "gene_symbol": "PRRC2A",
  "gene": "UniProtKB:P48634",
  "term_id": "GO:0030154"
}